caspase complex [GO:0008303] (cellular component) Note: Note that this term was reinstated from obsolete. Also known as: cysteine-type endopeptidase complex References: PMID:15569692 Sources: GOC:cna, GOC:mtg_apoptosis Definition: A protein complex that contains one or more cysteine-type endopeptidases (also called caspases), which give the complex a peptidase activity with specificity for the hydrolysis of aspartyl bonds. These complexes may be involved e.g. in apoptotic or inflammation processes. Relationships: is a type of endopeptidase complex [GO:1905369] Subtypes: GO:0042765, calpain complex [GO:0110158]